{
  "gene_symbol": "VPS11",
  "gene": "UniProtKB:Q9H270",
  "term_label": "protein-macromolecule adaptor activity",
  "term_id": "GO:0030674",
  "gene_name": "Vacuolar protein sorting-associated protein 11 homolog"
}